{
  "gene_symbol": "SNRPD1",
  "gene_name": "Small nuclear ribonucleoprotein Sm D1",
  "term_label": "spliceosomal snRNP assembly",
  "gene": "UniProtKB:P62314",
  "term_id": "GO:0000387"
}